{
  "term_label": "epigenetic programing of male pronucleus",
  "gene_name": "Protein STPG4",
  "gene_symbol": "STPG4",
  "gene": "UniProtKB:Q8N801",
  "term_id": "GO:0044727"
}